{
  "term_label": "positive regulation of phosphatidylinositol 3-kinase/protein kinase B signal transduction",
  "gene_name": "Guanine nucleotide exchange factor VAV2",
  "gene": "UniProtKB:P52735",
  "gene_symbol": "VAV2",
  "term_id": "GO:0051897"
}